(+)-secoisolariciresinol glucosyltransferase activity [GO:0102610] (molecular function) Definition: Catalysis of the reaction: (+)-secoisolariciresinol + UDP-alpha-D-glucose = (+)-secoisolariciresinol monoglucoside + UDP + H+. References: PMID:24678929 Sources: GOC:pz Relationships: is a type of hexosyltransferase activity [GO:0016758]